{
  "term_label": "glycine biosynthetic process from serine",
  "gene_symbol": "SHMT1",
  "gene_name": "Serine hydroxymethyltransferase, cytosolic",
  "gene": "UniProtKB:P34896",
  "term_id": "GO:0019264"
}